{
  "gene_name": "Ras-related protein Rab-6B",
  "gene_symbol": "RAB6B",
  "gene": "UniProtKB:Q9NRW1",
  "term_id": "GO:0006891",
  "term_label": "intra-Golgi vesicle-mediated transport"
}